{
  "term_id": "GO:0006954",
  "term_label": "inflammatory response",
  "gene_symbol": "PTGER2",
  "gene": "UniProtKB:P43116",
  "gene_name": "Prostaglandin E2 receptor EP2 subtype"
}